{
  "gene_symbol": "METAP1",
  "gene_name": "Methionine aminopeptidase 1",
  "term_id": "GO:0005829",
  "gene": "UniProtKB:P53582",
  "term_label": "cytosol"
}